peptidyl-D-alanine racemization [GO:0019122] (biological process) Relationships: is_a peptidyl-L-amino acid racemization [GO:0018085]; is a type of peptidyl-alanine modification [GO:0018194] Sources: RESID:AA0191 Also known as: alanine racemization Note: See also the biological process terms 'peptidyl-D-alanine racemization, direct ; GO:0019916' and 'peptidyl-D-alanine racemization via peptidyl-L-serine ; GO:0019917'. Definition: The formation of peptidyl-D-alanine, by either racemization or from peptidyl-L-serine.